{
  "gene": "UniProtKB:Q8WYK0",
  "term_label": "cytosol",
  "gene_symbol": "ACOT12",
  "gene_name": "Acetyl-coenzyme A thioesterase",
  "term_id": "GO:0005829"
}